{
  "gene": "UniProtKB:Q9H0U9",
  "term_label": "chromatin binding",
  "term_id": "GO:0003682",
  "gene_name": "Testis-specific Y-encoded-like protein 1",
  "gene_symbol": "TSPYL1"
}